anaerobic ribonucleoside-triphosphate reductase complex [GO:0031250] (cellular component) Definition: An enzyme complex composed of 4 subunits, 2 copies of the large protein (nrdD in E. coli) and 2 copies of the small protein (nrdG in E. coli). It catalyzes the generation of 2'deoxyribonucleotides under anaerobic growth conditions. The larger subunit is the catalytic unit that is activated by the smaller iron-binding subunit. Sources: GOC:mlg Relationships: is a type of catalytic complex [GO:1902494]; is part of GO:0005737